positive regulation of telomeric D-loop disassembly [GO:1905840] (biological process) Relationships: is a type of positive regulation of telomeric loop disassembly [GO:1904535]; is a type of regulation of telomeric D-loop disassembly [GO:1905838]; positively regulates telomeric D-loop disassembly [GO:0061820] Also known as: up regulation of telomeric D-loop disassembly, up-regulation of telomeric D-loop disassembly, upregulation of telomeric D-loop disassembly, activation of telomeric D-loop disassembly Definition: Any process that activates or increases the frequency, rate or extent of telomeric D-loop disassembly. References: PMID:15200954 Sources: GOC:BHF, GOC:BHF_telomere, GOC:TermGenie, GOC:nc, GO_REF:0000058